{
  "term_id": "UNKNOWN:0002",
  "term_label": "Unknown biological process",
  "gene_symbol": "OPALIN",
  "gene": "UniProtKB:Q96PE5",
  "gene_name": "Opalin"
}